crying behavior [GO:0060273] (biological process) Relationships: is a type of behavior [GO:0007610] Sources: GOC:dph Definition: The behavior in which an organism sheds tears, often accompanied by non-verbal vocalizations and in response to external or internal stimuli.